{
  "gene_symbol": "MAP1LC3B2",
  "term_id": "GO:0097352",
  "term_label": "autophagosome maturation",
  "gene_name": "Microtubule-associated proteins 1A_1B light chain 3 beta 2",
  "gene": "UniProtKB:A6NCE7"
}